{
  "gene_name": "Transmembrane protein 59",
  "gene": "UniProtKB:Q9BXS4",
  "gene_symbol": "TMEM59",
  "term_id": "GO:0010508",
  "term_label": "positive regulation of autophagy"
}